{
  "gene_symbol": "ADA",
  "gene": "UniProtKB:P00813",
  "gene_name": "Adenosine deaminase",
  "term_id": "GO:0043103",
  "term_label": "hypoxanthine salvage"
}